zinc ion import into Golgi lumen [GO:1904257] (biological process) Relationships: is a type of zinc ion import into organelle [GO:0062111]; is a type of cytosol to Golgi apparatus transport [GO:0140820] Also known as: cytosol to Golgi apparatus zinc transport, zinc II ion import across Golgi membrane, zinc ion import across Golgi membrane, zinc ion import into Golgi apparatus, zinc(2+) import across Golgi membrane, zinc ion import into Golgi membrane Definition: The directed import of zinc(2+) from the cytosol across the Golgi membrane into the Golgi lumen. References: PMID:25732056 Sources: GOC:TermGenie, GO_REF:0000075